{
  "term_label": "regulation of DNA-templated transcription",
  "term_id": "GO:0006355",
  "gene_symbol": "ZNF90",
  "gene_name": "Zinc finger protein 90",
  "gene": "UniProtKB:Q03938"
}